{
  "gene_name": "Myeloid-associated differentiation marker-like protein 2",
  "gene_symbol": "MYADML2",
  "gene": "UniProtKB:A6NDP7",
  "term_label": "Unknown cellular component",
  "term_id": "UNKNOWN:0003"
}